ureter maturation [GO:0035799] (biological process) Relationships: is a type of animal organ maturation [GO:0048799]; is part of ureter development [GO:0072189] Definition: A developmental process, independent of morphogenetic (shape) change, that is required for the ureter to attain its fully functional state. The ureter is a muscular tube that transports urine from the kidney to the urinary bladder or from the Malpighian tubule to the hindgut. References: PMID:17881463 Sources: GOC:bf, GOC:mtg_kidney_jan10, GOC:yaf